determination of pancreatic left/right asymmetry [GO:0035469] (biological process) References: PMID:12702646 Sources: GOC:dgh Definition: Determination of the asymmetric location of the pancreas with respect to the left and right halves of the organism. Relationships: is a type of determination of left/right symmetry [GO:0007368]; is part of pancreas development [GO:0031016]